viral DNA repair [GO:0046787] (biological process) Definition: The process of restoring viral DNA after damage or errors in replication. Relationships: is a type of DNA repair [GO:0006281]; is part of viral process [GO:0016032] Sources: ISBN:0781718325